DNA secretion by the type IV secretion system [GO:0044098] (biological process) Also known as: DNA secretion via the type IV secretion system Relationships: is a type of GO:0044097 Sources: GOC:pamgo_curators Definition: The controlled release of DNA by a cell, via the type IV secretion system.